{
  "gene": "UniProtKB:Q00796",
  "gene_name": "Sorbitol dehydrogenase",
  "term_label": "cytosol",
  "term_id": "GO:0005829",
  "gene_symbol": "SORD"
}